7,8-dihydropterin-6-yl-methyl-4-(beta-D-ribofuranosyl)aminobenzene 5'-phosphate synthase [GO:0102041] (molecular function) Sources: GOC:pz, RHEA:35951 Relationships: is a type of transferase activity, transferring alkyl or aryl (other than methyl) groups [GO:0016765] Definition: Catalysis of the reaction: 4-(beta-D-ribofuranosyl)aminobenzene 5'-phosphate + (2-amino-4-hydroxy-7,8-dihydropteridin-6-yl)methyl diphosphate = N-[(7,8-dihydropterin-6-yl)methyl]-4-(beta-D-ribofuranosyl)aniline 5'-phosphate + diphosphoric acid.